{
  "gene": "UniProtKB:A0A0B4J273",
  "gene_name": "T cell receptor alpha variable 34",
  "gene_symbol": "TRAV34",
  "term_label": "Unknown cellular component",
  "term_id": "UNKNOWN:0003"
}